NADPH phosphatase activity [GO:0102757] (molecular function) Relationships: is a type of phosphatase activity [GO:0016791] Definition: Catalysis of the reaction: NADPH + H2O = NADH + hydrogenphosphate. Sources: GOC:pz, RHEA:60664